{
  "gene_name": "C-C chemokine receptor type 4",
  "gene": "UniProtKB:P51679",
  "gene_symbol": "CCR4",
  "term_label": "positive regulation of cytosolic calcium ion concentration",
  "term_id": "GO:0007204"
}